N-formyl peptide receptor activity [GO:0004982] (molecular function) Also known as: Fmet-leu-phe receptor Sources: GOC:ai Definition: Combining with an N-formyl peptide to initiate a change in cell activity. Relationships: is a type of G protein-coupled peptide receptor activity [GO:0008528]